{
  "term_label": "mitochondrial inner membrane peptidase complex",
  "term_id": "GO:0042720",
  "gene_symbol": "IMMP1L",
  "gene": "UniProtKB:Q96LU5",
  "gene_name": "Mitochondrial inner membrane protease subunit 1"
}